{
  "term_id": "GO:0006357",
  "term_label": "regulation of transcription by RNA polymerase II",
  "gene_symbol": "E2F8",
  "gene_name": "Transcription factor E2F8",
  "gene": "UniProtKB:A0AVK6"
}